negative regulation of mitochondrial RNA catabolic process [GO:0000961] (biological process) Relationships: is a type of GO:0000960; is a type of negative regulation of RNA catabolic process [GO:1902369]; negatively regulates mitochondrial RNA catabolic process [GO:0000957] Subtypes: negative regulation of mitochondrial mRNA catabolic process [GO:1905638] Sources: GOC:krc, GOC:mah Definition: Any process that stops, prevents, or reduces the frequency, rate or extent of the chemical reactions and pathways involving catabolism in the mitochondrion of RNA transcribed from the mitochondrial genome.